{
  "gene_name": "Phosphoglycerate kinase 2",
  "gene_symbol": "PGK2",
  "gene": "UniProtKB:P07205",
  "term_id": "GO:0035686",
  "term_label": "sperm fibrous sheath"
}